{
  "term_label": "DNA-binding transcription repressor activity, RNA polymerase II-specific",
  "gene": "UniProtKB:Q9HBE1",
  "term_id": "GO:0001227",
  "gene_name": "POZ-, AT hook-, and zinc finger-containing protein 1",
  "gene_symbol": "PATZ1"
}